negative regulation of phosphatidylserine biosynthetic process [GO:1900469] (biological process) Relationships: is a type of negative regulation of phospholipid biosynthetic process [GO:0071072]; is a type of regulation of phosphatidylserine biosynthetic process [GO:1900468]; negatively regulates phosphatidylserine biosynthetic process [GO:0006659] Definition: Any process that stops, prevents or reduces the frequency, rate or extent of phosphatidylserine biosynthetic process. Also known as: down regulation of phosphatidylserine anabolism, down regulation of phosphatidylserine biosynthesis, down regulation of phosphatidylserine biosynthetic process, down regulation of phosphatidylserine formation, down regulation of phosphatidylserine synthesis, down-regulation of phosphatidylserine anabolism, down-regulation of phosphatidylserine biosynthesis, down-regulation of phosphatidylserine biosynthetic process, down-regulation of phosphatidylserine formation, down-regulation of phosphatidylserine synthesis, downregulation of phosphatidylserine anabolism, downregulation of phosphatidylserine biosynthesis, downregulation of phosphatidylserine biosynthetic process, downregulation of phosphatidylserine formation, downregulation of phosphatidylserine synthesis, inhibition of phosphatidylserine anabolism, inhibition of phosphatidylserine biosynthesis, inhibition of phosphatidylserine formation, inhibition of phosphatidylserine synthesis, negative regulation of phosphatidylserine anabolism, negative regulation of phosphatidylserine biosynthesis, negative regulation of phosphatidylserine formation, negative regulation of phosphatidylserine synthesis, inhibition of phosphatidylserine biosynthetic process References: PMID:8056324, PMID:8614637 Sources: GOC:TermGenie, GOC:dgf